{
  "term_label": "Unknown molecular function",
  "gene_name": "Caspase recruitment domain-containing protein 18",
  "gene": "UniProtKB:P57730",
  "term_id": "UNKNOWN:0001",
  "gene_symbol": "CARD18"
}